{
  "gene": "UniProtKB:P17066",
  "term_id": "GO:0031072",
  "gene_name": "Heat shock 70 kDa protein 6",
  "gene_symbol": "HSPA6",
  "term_label": "heat shock protein binding"
}